{
  "gene_name": "BET1 homolog",
  "term_id": "GO:0005484",
  "gene": "UniProtKB:O15155",
  "term_label": "SNAP receptor activity",
  "gene_symbol": "BET1"
}